{
  "gene": "UniProtKB:B2RXH2",
  "gene_symbol": "KDM4E",
  "gene_name": "Lysine-specific demethylase 4E",
  "term_id": "GO:0000785",
  "term_label": "chromatin"
}